{
  "gene_name": "Zinc finger protein 707",
  "term_id": "GO:0006357",
  "term_label": "regulation of transcription by RNA polymerase II",
  "gene_symbol": "ZNF707",
  "gene": "UniProtKB:Q96C28"
}